{
  "gene_symbol": "A6NJR5",
  "gene_name": "Putative speedy protein-like protein 3",
  "term_label": "Unknown biological process",
  "gene": "UniProtKB:A6NJR5",
  "term_id": "UNKNOWN:0002"
}